{
  "gene_symbol": "CAP1",
  "gene": "UniProtKB:Q01518",
  "term_label": "cytoplasm",
  "gene_name": "Adenylyl cyclase-associated protein 1",
  "term_id": "GO:0005737"
}